rumination [GO:0036147] (BP) Relationships: is a type of digestive system process [GO:0022600] Definition: A digestive process in which food, usually grass or hay, is swallowed into a multi-compartmented stomach, regurgitated, chewed again, and swallowed again. Also known as: digestive rumination Sources: GOC:maf, Wikipedia:Rumination